{
  "term_label": "calcineurin complex",
  "gene_name": "Serine_threonine-protein phosphatase 2B catalytic subunit gamma isoform",
  "gene_symbol": "PPP3CC",
  "term_id": "GO:0005955",
  "gene": "UniProtKB:P48454"
}